{
  "gene_name": "Tetra-peptide repeat homeobox protein 1",
  "gene": "UniProtKB:Q8N7U7",
  "term_label": "Unknown biological process",
  "term_id": "UNKNOWN:0002",
  "gene_symbol": "TPRX1"
}